{
  "term_label": "proteolysis",
  "gene": "UniProtKB:P59510",
  "gene_symbol": "ADAMTS20",
  "gene_name": "A disintegrin and metalloproteinase with thrombospondin motifs 20",
  "term_id": "GO:0006508"
}